{
  "term_id": "GO:0006643",
  "gene_name": "Alkylglycerol monooxygenase",
  "term_label": "membrane lipid metabolic process",
  "gene_symbol": "AGMO",
  "gene": "UniProtKB:Q6ZNB7"
}